{
  "gene_symbol": "TLR4",
  "term_id": "GO:0001530",
  "gene_name": "Toll-like receptor 4",
  "gene": "UniProtKB:O00206",
  "term_label": "lipopolysaccharide binding"
}